interleukin-12 production [GO:0032615] (biological process) Also known as: IL-12 production, CLMF production, NKSF production, interleukin-12 biosynthetic process, interleukin-12 secretion Sources: GOC:mah Regulation: regulated by regulation of interleukin-12 production [GO:0032655]; negatively regulated by negative regulation of interleukin-12 production [GO:0032695]; positively regulated by GO:0032735 Definition: The appearance of interleukin-12 due to biosynthesis or secretion following a cellular stimulus, resulting in an increase in its intracellular or extracellular levels. Relationships: is a type of cytokine production [GO:0001816]